regulatory ncRNA-mediated gene silencing [GO:0031047] (biological process) Definition: A process in which an regulatory non-coding RNA molecule reduces expression of target genes. This can occur pre-transcriptionally by assembly of heterochromatin and prevention of transcription or co- or post-transcriptionally by targeting RNAs for degradation or by interfering with splicing or translation. This process starts once the inhibitory RNA molecule has been transcribed, and includes processing of the RNA such as cleavage, modifications, transport from the nucleus to the cytoplasm, loading onto the RISC complex, and the effect on transcription or translation. References: PMID:15020054 Also known as: RNA-dependent gene silencing, RNA-mediated gene silencing, gene silencing by RNA Relationships: is a type of negative regulation of gene expression [GO:0010629] Subtypes: regulatory ncRNA-mediated heterochromatin formation [GO:0031048], co-transcriptional gene silencing by RNA interference machinery [GO:0033562], regulatory ncRNA-mediated post-transcriptional gene silencing [GO:0035194] Regulation: regulated by regulation of gene silencing by regulatory ncRNA [GO:0060966]; negatively regulated by negative regulation of gene silencing by regulatory ncRNA [GO:0060967]